proximal convoluted tubule segment 1 cell development [GO:0072145] (BP) Definition: The process whose specific outcome is the progression of an S1 cell in the kidney over time, from its formation to the mature structure. Also known as: S1 cell development Sources: GOC:bf, GOC:mtg_kidney_jan10 Relationships: is a type of cell development [GO:0048468]; is part of proximal convoluted tubule segment 1 cell differentiation [GO:0072062]